{
  "term_label": "actomyosin",
  "term_id": "GO:0042641",
  "gene": "UniProtKB:Q5VT25",
  "gene_symbol": "CDC42BPA",
  "gene_name": "Serine_threonine-protein kinase MRCK alpha"
}